{
  "gene_name": "Protein FAM236A",
  "term_id": "UNKNOWN:0002",
  "gene": "UniProtKB:A0A1B0GUQ0",
  "term_label": "Unknown biological process",
  "gene_symbol": "FAM236A"
}